isoflavone-7-O-beta-glucoside 6''-O-malonyltransferase activity [GO:0047164] (molecular function) Sources: EC:2.3.1.115 Also known as: MAT-7, flavone (flavonol) 7-O-glycoside malonyltransferase activity, flavone/flavonol 7-O-beta-D-glucoside malonyltransferase activity, malonyl-CoA:flavone/flavonol 7-O-glucoside malonyltransferase activity, malonyl-CoA:isoflavone-7-O-beta-D-glucoside 6''-O-malonyltransferase activity, malonyl-coenzyme A:flavone/flavonol-7-O-glycoside malonyltransferase activity, malonyl-coenzyme A:isoflavone 7-O-glucoside-6''-malonyltransferase activity Relationships: is a type of GO:0050736 Definition: Catalysis of the reaction: biochanin-A + malonyl-CoA = 6'-malonyl-biochanin A + CoA.